regulation of synaptic vesicle recycling [GO:1903421] (biological process) Relationships: is a type of regulation of transport [GO:0051049]; regulates synaptic vesicle recycling [GO:0036465] Note: An example of this is mouse LRRK2 (Q5S006) in PMID:21307259 inferred from mutant phenotype Definition: Any process that modulates the frequency, rate or extent of synaptic vesicle recycling. Also known as: regulation of kiss-and-run synaptic vesicle recycling, regulation of kiss-and-stay synaptic vesicle recycling References: PMID:22745285 Sources: GOC:PARL, GOC:TermGenie, GOC:pad, GO_REF:0000058 Subtypes: regulation of recycling endosome localization within postsynapse [GO:0099158], regulation of synaptic vesicle endocytosis [GO:1900242], GO:1903422, positive regulation of synaptic vesicle recycling [GO:1903423]